{
  "term_id": "GO:0060633",
  "gene": "UniProtKB:Q9Y4E5",
  "gene_symbol": "ZNF451",
  "gene_name": "E3 SUMO-protein ligase ZNF451",
  "term_label": "negative regulation of transcription initiation by RNA polymerase II"
}